{
  "gene_symbol": "SIK1",
  "gene_name": "Serine_threonine-protein kinase SIK1",
  "term_id": "GO:0035556",
  "gene": "UniProtKB:P57059",
  "term_label": "intracellular signal transduction"
}